medium-chain fatty acid transport [GO:0001579] (BP) Sources: GOC:ai Definition: The directed movement of a medium-chain fatty acid into, out of or within a cell, or between cells, by means of some agent such as a transporter or pore. A medium-chain fatty acid has an aliphatic tail containing 6 to 12 carbons. Note: While there is not universal consensus on the lengths of short-, medium-, long- and very-long-chain fatty acids, the GO uses the definitions in ChEBI (see CHEBI:26666, CHEBI:59554, CHEBI:15904 and CHEBI:27283). Relationships: is a type of fatty acid transport [GO:0015908]